{
  "gene_symbol": "PRDX2",
  "term_id": "GO:0005829",
  "gene_name": "Peroxiredoxin-2",
  "term_label": "cytosol",
  "gene": "UniProtKB:P32119"
}